{
  "term_id": "GO:0005634",
  "term_label": "nucleus",
  "gene_name": "Myeloid leukemia factor 1",
  "gene_symbol": "MLF1",
  "gene": "UniProtKB:P58340"
}